{
  "gene_symbol": "PSMD12",
  "term_label": "Unknown biological process",
  "gene": "UniProtKB:O00232",
  "term_id": "UNKNOWN:0002",
  "gene_name": "26S proteasome non-ATPase regulatory subunit 12"
}